microvillus [GO:0005902] (CC) Relationships: is a type of GO:0098858; has part actin filament bundle [GO:0032432] Note: Note that this term refers to a projection from a single cell, and should not be confused with 'microvillus' as used to refer to a multicellular structure such as that found in the placenta. Sources: ISBN:0815316194 Also known as: microvilli Subtypes: rhabdomere microvillus [GO:0035996], Schwann cell microvillus [GO:0097454] Definition: Thin cylindrical membrane-covered projections on the surface of an animal cell containing a core bundle of actin filaments. Present in especially large numbers on the absorptive surface of intestinal cells.